lipopolysaccharide transport [GO:0015920] (biological process) Also known as: LPS transport, LPS export, lipopolysaccharide export Definition: The directed movement of lipopolysaccharides into, out of or within a cell, or between cells, by means of some agent such as a transporter or pore. A lipopolysaccharide is any of a group of related, structurally complex components of the outer membrane of Gram-negative bacteria. Lipopolysaccharides consist three covalently linked regions, lipid A, core oligosaccharide, and an O side chain. Lipid A is responsible for the toxicity of the lipopolysaccharide. Relationships: is_a GO:0006869; is a type of GO:1901264 Sources: GOC:ai